all-trans retinal binding [GO:0005503] (molecular function) Relationships: is a type of retinal binding [GO:0016918] Also known as: vitamin A binding, all-trans retinaldehyde binding, trans retinal binding, visual yellow binding, xanthopsin Definition: Binding to all-trans retinal, a compound that plays an important role in the visual process in most vertebrates. All-trans retinal (trans r., visual yellow) results from the bleaching of rhodopsin by light, in which the 11-cis form is converted to the all-trans form. Retinal is one of the forms of vitamin A. Sources: GOC:curators